MDA-5 signaling pathway [GO:0039530] (biological process) Relationships: is a type of cytoplasmic pattern recognition receptor signaling pathway [GO:0002753] References: PMID:19620789, PMID:33087405 Sources: GOC:bf Also known as: IFIH1 signaling pathway, MDA-5 signalling pathway, melanoma differentiation-associated gene 5 signaling pathway, MDA5 signaling pathway Definition: The series of molecular signals initiated by the binding of dsRNA from another organism to the cytoplasmic pattern recognition receptor (PRR) MDA-5 (also known as IFIH1). MDA-5 detects RNA synthesized during viral replication or shed by non-viral pathogens, and triggers a signaling pathway to protect the host against infection, for example by inducing the expression of cytokines. Regulation: regulated by regulation of MDA-5 signaling pathway [GO:0039533]; negatively regulated by negative regulation of MDA-5 signaling pathway [GO:0039534]; positively regulated by positive regulation of MDA-5 signaling pathway [GO:1900245]